{
  "gene_name": "Tether containing UBX domain for GLUT4",
  "term_label": "vesicle membrane",
  "gene": "UniProtKB:Q9BZE9",
  "gene_symbol": "ASPSCR1",
  "term_id": "GO:0012506"
}